fructose uniporter activity [GO:0015284] (molecular function) Relationships: is a type of fructose transmembrane transporter activity [GO:0005353]; is a type of hexose uniporter activity [GO:0008516] Sources: TC:2.A.1.1.13 Definition: Enables the transfer of a solute or solutes from one side of a membrane to the other according to the reaction: fructose(out) = fructose(in).